{
  "gene_name": "A disintegrin and metalloproteinase with thrombospondin motifs 14",
  "gene_symbol": "ADAMTS14",
  "gene": "UniProtKB:Q8WXS8",
  "term_label": "extracellular matrix",
  "term_id": "GO:0031012"
}